{
  "gene_symbol": "SLC12A7",
  "term_label": "plasma membrane",
  "term_id": "GO:0005886",
  "gene": "UniProtKB:Q9Y666",
  "gene_name": "Solute carrier family 12 member 7"
}